{
  "gene_name": "Zinc finger protein 787",
  "gene_symbol": "ZNF787",
  "term_label": "sequence-specific DNA binding",
  "term_id": "GO:0043565",
  "gene": "UniProtKB:Q6DD87"
}